apelin receptor signaling pathway [GO:0060183] (BP) Definition: A G protein-coupled receptor signaling pathway initiated by apelin binding to its receptor on the surface of a target cell, and ending with the regulation of a downstream cellular process. Sources: GOC:dph Also known as: apelin receptor signalling pathway Relationships: is a type of G protein-coupled receptor signaling pathway [GO:0007186]